{
  "gene_symbol": "STK32A",
  "term_label": "intracellular signal transduction",
  "gene_name": "Serine_threonine-protein kinase 32A",
  "term_id": "GO:0035556",
  "gene": "UniProtKB:Q8WU08"
}